symbiont entry into host cell via disruption of host cell wall peptidoglycan [GO:0098932] (biological process) Sources: GOC:dos, VZ:3940 Also known as: catabolism of host cell wall peptidoglycan by virus, degradation of host cell wall peptidoglycan by virus, degradation of host peptidoglycans during virus entry, disassembly by virus of host cell wall peptidoglycan, disruption by virus of host cell wall peptidoglycan during virus entry Definition: The disruption by a symbiont of host cell wall peptidoglycans to allow entry into the host cell. Relationships: is a type of GO:0052009; is part of symbiont entry into host cell [GO:0046718]